cellular response to hesperadin [GO:0072763] (biological process) Definition: Any process that results in a change in state or activity of a cell (in terms of movement, secretion, enzyme production, gene expression, etc.) as a result of a hesperadin stimulus. Relationships: is a type of cellular response to amine stimulus [GO:0071418]; is a type of response to hesperadin [GO:1901595]; is a type of cellular response to oxygen-containing compound [GO:1901701] Sources: GOC:mah